{
  "term_id": "GO:0051664",
  "gene_name": "Lamin-B2",
  "term_label": "nuclear pore localization",
  "gene": "UniProtKB:Q03252",
  "gene_symbol": "LMNB2"
}